{
  "term_label": "cilium organization",
  "gene_symbol": "MNS1",
  "gene_name": "Meiosis-specific nuclear structural protein 1",
  "gene": "UniProtKB:Q8NEH6",
  "term_id": "GO:0044782"
}